indole 2,3-dioxygenase activity [GO:0047719] (molecular function) Sources: EC:1.13.11.17, RHEA:11212 Relationships: is a type of oxidoreductase activity, acting on single donors with incorporation of molecular oxygen, incorporation of two atoms of oxygen [GO:0016702] Also known as: IDO, indole oxidase activity, indole-oxygen 2,3-oxidoreductase (decyclizing), indole:O2 oxidoreductase activity, indole:oxygen 2,3-oxidoreductase (decyclizing) Definition: Catalysis of the reaction: indole + O2 = 2-formamidobenzaldehyde.